{
  "term_label": "Unknown molecular function",
  "gene": "UniProtKB:Q9NS86",
  "term_id": "UNKNOWN:0001",
  "gene_symbol": "LANCL2",
  "gene_name": "LanC-like protein 2"
}